{
  "gene_symbol": "IL32",
  "gene": "UniProtKB:P24001",
  "gene_name": "Interleukin-32",
  "term_label": "Unknown molecular function",
  "term_id": "UNKNOWN:0001"
}